{
  "gene_name": "Calcium-binding protein 2",
  "gene": "UniProtKB:Q9NPB3",
  "term_id": "GO:0005886",
  "term_label": "plasma membrane",
  "gene_symbol": "CABP2"
}